{
  "gene_symbol": "PGC",
  "term_id": "GO:0005615",
  "term_label": "extracellular space",
  "gene_name": "Gastricsin",
  "gene": "UniProtKB:P20142"
}